{
  "term_id": "GO:0004222",
  "gene_name": "Neutrophil collagenase",
  "term_label": "metalloendopeptidase activity",
  "gene_symbol": "MMP8",
  "gene": "UniProtKB:P22894"
}